{
  "term_label": "RNA polymerase II core complex assembly",
  "gene": "UniProtKB:Q00403",
  "gene_name": "Transcription initiation factor IIB",
  "gene_symbol": "GTF2B",
  "term_id": "GO:1990114"
}